{
  "term_label": "immunoglobulin complex",
  "gene_name": "Immunoglobulin lambda variable 3-10",
  "gene": "UniProtKB:A0A075B6K4",
  "term_id": "GO:0019814",
  "gene_symbol": "IGLV3-10"
}